{
  "gene_symbol": "U2AF2",
  "term_label": "commitment complex",
  "gene": "UniProtKB:P26368",
  "term_id": "GO:0000243",
  "gene_name": "Splicing factor U2AF 65 kDa subunit"
}